{
  "gene_name": "26S proteasome non-ATPase regulatory subunit 1",
  "gene": "UniProtKB:Q99460",
  "term_id": "GO:0043161",
  "gene_symbol": "PSMD1",
  "term_label": "proteasome-mediated ubiquitin-dependent protein catabolic process"
}